{
  "gene": "UniProtKB:O43150",
  "gene_symbol": "ASAP2",
  "term_label": "plasma membrane",
  "gene_name": "Arf-GAP with SH3 domain, ANK repeat and PH domain-containing protein 2",
  "term_id": "GO:0005886"
}